{
  "term_label": "synaptic vesicle membrane",
  "term_id": "GO:0030672",
  "gene_name": "Synaptic vesicle glycoprotein 2A",
  "gene": "UniProtKB:Q7L0J3",
  "gene_symbol": "SV2A"
}